{
  "term_label": "microtubule-based movement",
  "gene_name": "Kinesin-like protein KIF18B",
  "gene": "UniProtKB:Q86Y91",
  "gene_symbol": "KIF18B",
  "term_id": "GO:0007018"
}